{
  "gene_name": "Angiogenic factor with G patch and FHA domains 1",
  "gene_symbol": "AGGF1",
  "term_id": "GO:0045766",
  "gene": "UniProtKB:Q8N302",
  "term_label": "positive regulation of angiogenesis"
}